myofibroblast differentiation [GO:0036446] (biological process) Definition: The process in which an undifferentiated cell acquires the features of a myofibroblast cell. Regulation: regulated by regulation of myofibroblast differentiation [GO:1904760]; negatively regulated by negative regulation of myofibroblast differentiation [GO:1904761]; positively regulated by GO:1904762 Also known as: myofibroblast cell differentiation Sources: CL:0000186, GOC:nhn Relationships: is a type of cell differentiation [GO:0030154]